{
  "gene_name": "Glycine dehydrogenase (decarboxylating), mitochondrial",
  "gene": "UniProtKB:P23378",
  "term_label": "glycine cleavage complex",
  "term_id": "GO:0005960",
  "gene_symbol": "GLDC"
}